{
  "term_label": "retrograde vesicle-mediated transport, Golgi to endoplasmic reticulum",
  "gene_name": "Vesicle transport protein USE1",
  "term_id": "GO:0006890",
  "gene": "UniProtKB:Q9NZ43",
  "gene_symbol": "USE1"
}